2-aminobenzenesulfonate desulfonation [GO:0019490] (biological process) Relationships: is a type of 2-aminobenzenesulfonate catabolic process [GO:0046230] Also known as: 2-aminobenzenesulphonate desulphonation Definition: The removal of the sulfonate group from 2-aminobenzenesulfonate, an aromatic sulfonate used in organic synthesis and in the manufacture of various dyes and medicines. Sources: MetaCyc:2ASDEG-PWY